{
  "gene": "UniProtKB:P11597",
  "gene_symbol": "CETP",
  "term_label": "high-density lipoprotein particle remodeling",
  "gene_name": "Cholesteryl ester transfer protein",
  "term_id": "GO:0034375"
}